positive regulation of wax biosynthetic process [GO:1904278] (biological process) Relationships: is a type of positive regulation of lipid biosynthetic process [GO:0046889]; is a type of regulation of wax biosynthetic process [GO:1904276]; positively regulates GO:0010025 Definition: Any process that activates or increases the frequency, rate or extent of wax biosynthetic process. References: PMID:24692420 Sources: GOC:TermGenie, GO_REF:0000058 Also known as: positive regulation of wax anabolism, positive regulation of wax biosynthesis, positive regulation of wax formation, positive regulation of wax synthesis, up regulation of wax anabolism, up regulation of wax biosynthesis, up regulation of wax biosynthetic process, up regulation of wax formation, up regulation of wax synthesis, up-regulation of wax anabolism, up-regulation of wax biosynthesis, up-regulation of wax biosynthetic process, up-regulation of wax formation, up-regulation of wax synthesis, upregulation of wax anabolism, upregulation of wax biosynthesis, upregulation of wax biosynthetic process, upregulation of wax formation, upregulation of wax synthesis, activation of wax anabolism, activation of wax biosynthesis, activation of wax biosynthetic process, activation of wax formation, activation of wax synthesis